Fc-epsilon receptor I complex [GO:0032998] (cellular component) Definition: A protein complex composed of an Fc-epsilon RI alpha chain and an Fc-epsilon RI gamma chain dimer with or without an Fc-episilon RI beta chain and additional signaling components. The complex functions primarily as an activating receptor for IgE. Sources: GOC:add, ISBN:0781735149 Relationships: is a type of Fc receptor complex [GO:0032997] Also known as: IgE receptor complex, immunoglobulin E receptor complex, FceRI complex